hexameric IgM immunoglobulin complex [GO:0071757] (cellular component) Definition: A circulating form of IgM consisting of a hexamer of IgM core units with a single J chain polypeptide. References: PMID:20176268 Sources: GOC:add, ISBN:0781765196 Also known as: hexameric IgM antibody Note: Note that an IgM immunoglobulin complex has the function of antigen binding if a suitable antigen is available. Relationships: is a type of IgM immunoglobulin complex, circulating [GO:0071754]